{
  "gene_symbol": "H3-4",
  "term_label": "nucleosomal DNA binding",
  "gene_name": "Histone H3.1t",
  "gene": "UniProtKB:Q16695",
  "term_id": "GO:0031492"
}